{
  "gene_name": "Mitogen-activated protein kinase kinase kinase 1",
  "gene": "UniProtKB:Q13233",
  "term_label": "MAPK cascade",
  "term_id": "GO:0000165",
  "gene_symbol": "MAP3K1"
}